{
  "term_label": "C-C chemokine receptor activity",
  "gene_symbol": "CXCR1",
  "gene_name": "C-X-C chemokine receptor type 1",
  "term_id": "GO:0016493",
  "gene": "UniProtKB:P25024"
}